{
  "gene_name": "Rhomboid-related protein 3",
  "term_label": "Unknown biological process",
  "gene_symbol": "RHBDL3",
  "gene": "UniProtKB:P58872",
  "term_id": "UNKNOWN:0002"
}